inosine salvage [GO:0006190] (biological process) Relationships: is a type of purine ribonucleoside salvage [GO:0006166]; is a type of inosine biosynthetic process [GO:0046103] Sources: GOC:jl Also known as: adenine, hypoxanthine and their nucleoside salvage, guanine, xanthine and their nucleoside salvage Definition: Any process that generates inosine, hypoxanthine riboside, from derivatives of it without de novo synthesis.